{
  "term_label": "Unknown biological process",
  "gene_symbol": "SBF1",
  "gene": "UniProtKB:O95248",
  "gene_name": "Myotubularin-related protein 5",
  "term_id": "UNKNOWN:0002"
}